{
  "gene": "UniProtKB:Q8WW12",
  "gene_symbol": "PCNP",
  "term_label": "Unknown molecular function",
  "term_id": "UNKNOWN:0001",
  "gene_name": "PEST proteolytic signal-containing nuclear protein"
}